acetyl-CoA biosynthetic process from acetate [GO:0019427] (biological process) Sources: MetaCyc:ACETATEUTIL-PWY Also known as: acetyl-CoA anabolism from acetate, acetyl-CoA formation from acetate, acetyl-CoA synthesis from acetate, acetate utilization Definition: The chemical reactions and pathways resulting in the formation of acetyl-CoA from acetate, either directly or via acetylphosphate. Relationships: is a type of GO:0006083; is a type of acetyl-CoA biosynthetic process [GO:0006085]